{
  "term_id": "UNKNOWN:0002",
  "gene": "UniProtKB:A0A075B6Y8",
  "gene_name": "T cell receptor alpha joining 11 (Fragment)",
  "gene_symbol": "TRAJ11",
  "term_label": "Unknown biological process"
}